regulation of prolactin signaling pathway [GO:1902211] (biological process) Definition: Any process that modulates the frequency, rate or extent of prolactin signaling pathway. Also known as: regulation of PRL signaling pathway, regulation of prolactin-mediated signaling pathway References: PMID:11773439 Sources: GOC:TermGenie Relationships: is a type of regulation of cytokine-mediated signaling pathway [GO:0001959]; regulates prolactin signaling pathway [GO:0038161] Subtypes: negative regulation of prolactin signaling pathway [GO:1902212], positive regulation of prolactin signaling pathway [GO:1902213]